{
  "gene": "UniProtKB:O00451",
  "term_id": "GO:0043235",
  "term_label": "receptor complex",
  "gene_symbol": "GFRA2",
  "gene_name": "GDNF family receptor alpha-2"
}